{
  "gene": "UniProtKB:Q8N9G6",
  "term_label": "Unknown biological process",
  "gene_name": "Putative UPF0607 protein FLJ37424",
  "gene_symbol": "Q8N9G6",
  "term_id": "UNKNOWN:0002"
}